{
  "gene_name": "Moesin",
  "term_label": "regulation of organelle assembly",
  "gene_symbol": "MSN",
  "term_id": "GO:1902115",
  "gene": "UniProtKB:P26038"
}